{
  "gene": "UniProtKB:Q02447",
  "term_label": "nucleus",
  "gene_symbol": "SP3",
  "term_id": "GO:0005634",
  "gene_name": "Transcription factor Sp3"
}